{
  "term_id": "UNKNOWN:0003",
  "term_label": "Unknown cellular component",
  "gene_symbol": "CFAP97",
  "gene_name": "Cilia- and flagella-associated protein 97",
  "gene": "UniProtKB:Q9P2B7"
}